{
  "gene": "UniProtKB:O75112",
  "term_label": "adherens junction",
  "gene_name": "LIM domain-binding protein 3",
  "term_id": "GO:0005912",
  "gene_symbol": "LDB3"
}